Casparian strip assembly [GO:0160073] (biological process) Also known as: Casparian strip formation Relationships: is a type of cellular component assembly [GO:0022607]; is part of plant-type cell wall assembly [GO:0071668] Definition: The aggregation, arrangement and bonding together of a set of components to form a Casparian strip, a region of plant cell wall specialised to act as a seal to prevent back leakage of secreted material. References: PMID:28104889